{
  "gene": "UniProtKB:O14786",
  "term_id": "GO:0005886",
  "gene_name": "Neuropilin-1",
  "term_label": "plasma membrane",
  "gene_symbol": "NRP1"
}